{
  "term_label": "positive regulation of sodium ion export across plasma membrane",
  "gene_name": "FXYD domain-containing ion transport regulator 4",
  "term_id": "GO:1903278",
  "gene": "UniProtKB:P59646",
  "gene_symbol": "FXYD4"
}